iron-sulfur-molybdenum cofactor assembly [GO:0044593] (biological process) References: PMID:18429691 Sources: GOC:mengo_curators, GOC:tt Definition: The chemical reactions and pathways resulting in the formation of iron-sulfur-molybdenum cofactor, the cofactor located at the active site of the molybdenum nitrogenase. Regulation: regulated by GO:1900506; negatively regulated by GO:1900507; positively regulated by positive regulation of iron-sulfur-molybdenum cofactor assembly [GO:1900508] Also known as: FeMoco assembly, FeMoco biosynthetic process, iron molybdenum cofactor assembly, iron molybdenum cofactor biosynthesis, iron molybdenum cofactor biosynthetic process Relationships: is a type of iron-sulfur cluster assembly [GO:0016226]